{
  "gene_name": "Peptidyl-prolyl cis-trans isomerase H",
  "gene": "UniProtKB:O43447",
  "gene_symbol": "PPIH",
  "term_label": "cyclosporin A binding",
  "term_id": "GO:0016018"
}